{
  "term_label": "fusion of sperm to egg plasma membrane involved in single fertilization",
  "gene_symbol": "LYZL4",
  "gene": "UniProtKB:Q96KX0",
  "gene_name": "Lysozyme-like protein 4",
  "term_id": "GO:0007342"
}